{
  "term_id": "GO:0036158",
  "gene_name": "Dynein axonemal intermediate chain 2",
  "gene_symbol": "DNAI2",
  "gene": "UniProtKB:Q9GZS0",
  "term_label": "outer dynein arm assembly"
}